{
  "gene_name": "Retinal rod rhodopsin-sensitive cGMP 3',5'-cyclic phosphodiesterase subunit delta",
  "gene_symbol": "PDE6D",
  "term_id": "GO:0005737",
  "gene": "UniProtKB:O43924",
  "term_label": "cytoplasm"
}